allantoin:proton symporter activity [GO:0005274] (molecular function) Definition: Enables the transfer of a solute or solutes from one side of a membrane to the other according to the reaction: allantoin(out) + H+(out) = allantoin(in) + H+(in) by secondary active transport. Sources: GOC:mtg_transport, ISBN:0815340729, TC:2.A.39.3.1 Relationships: is a type of solute:proton symporter activity [GO:0015295]; is a type of GO:0042887; is part of allantoin transport [GO:0015720] Also known as: allantoin/allantoate transporter, allantoin uptake transmembrane transporter activity, allantoin permease activity